{
  "gene_symbol": "EFL1",
  "term_id": "GO:1990904",
  "gene": "UniProtKB:Q7Z2Z2",
  "gene_name": "Elongation factor-like GTPase 1",
  "term_label": "ribonucleoprotein complex"
}